pantothenate:sodium symporter activity [GO:0015498] (molecular function) Definition: Enables the transfer of a solute or solutes from one side of a membrane to the other according to the reaction: pantothenate(out) + Na+(out) = pantothenate(in) + Na+(in). Relationships: is a type of GO:0005343; is a type of amide transmembrane transporter activity [GO:0042887]; is_a carboxylic acid transmembrane transporter activity [GO:0046943]; is a type of modified amino acid transmembrane transporter activity [GO:0072349]; is part of sodium ion import across plasma membrane [GO:0098719] Sources: TC:2.A.21.1.1